negative regulation of viral budding via host ESCRT complex [GO:1903773] (biological process) Relationships: is a type of regulation of viral budding via host ESCRT complex [GO:1903772]; is a type of negative regulation of viral life cycle [GO:1903901]; negatively regulates viral budding via host ESCRT complex [GO:0039702] References: PMID:24878737 Sources: GOC:TermGenie, GOC:als, GO_REF:0000058 Also known as: down regulation of viral budding via host ESCRT complex, down-regulation of viral budding via host ESCRT complex, downregulation of viral budding via host ESCRT complex, inhibition of viral budding via host ESCRT complex, down regulation of viral budding through the ESCRT machinery, down-regulation of viral budding through the ESCRT machinery, downregulation of viral budding through the ESCRT machinery, inhibition of viral budding through the ESCRT machinery, negative regulation of viral budding through the ESCRT machinery Definition: Any process that stops, prevents or reduces the frequency, rate or extent of viral budding via host ESCRT complex.